{
  "gene": "UniProtKB:O14746",
  "term_label": "telomere maintenance via telomerase",
  "term_id": "GO:0007004",
  "gene_name": "Telomerase reverse transcriptase",
  "gene_symbol": "TERT"
}